{
  "term_id": "GO:0015183",
  "gene": "UniProtKB:Q9H1K4",
  "gene_name": "Mitochondrial glutamate carrier 2",
  "gene_symbol": "SLC25A18",
  "term_label": "L-aspartate transmembrane transporter activity"
}